reproductive shoot system development [GO:0090567] (biological process) Definition: The process whose specific outcome is the progression of a reproductive shoot system over time, from its formation to the mature structure. Subtypes: GO:0009908, inflorescence development [GO:0010229] Sources: GOC:pj Relationships: is_a post-embryonic development [GO:0009791]; is_a GO:0048367; is a type of reproductive structure development [GO:0048608]